establishment of skin barrier [GO:0061436] (biological process) Definition: Establishment of the epithelial barrier, the functional barrier in the skin that limits its permeability. Sources: GOC:dph Relationships: is a type of skin epidermis development [GO:0098773] Also known as: establishment of epithelial barrier, epithelial barrier development, skin barrier development